{
  "gene_name": "Polycomb protein SCMH1",
  "term_id": "GO:0005634",
  "gene_symbol": "SCMH1",
  "term_label": "nucleus",
  "gene": "UniProtKB:Q96GD3"
}